{
  "gene_symbol": "NPW",
  "term_id": "UNKNOWN:0003",
  "gene": "UniProtKB:Q8N729",
  "term_label": "Unknown cellular component",
  "gene_name": "Neuropeptide W"
}